regulation of behavior [GO:0050795] (biological process) Sources: GOC:go_curators, GOC:pr Definition: Any process that modulates the frequency, rate or extent of behavior, the internally coordinated responses (actions or inactions) of whole living organisms (individuals or groups) to internal or external stimuli. Relationships: is a type of regulation of multicellular organismal process [GO:0051239]; regulates behavior [GO:0007610] Also known as: regulation of behaviour Subtypes: regulation of host-seeking behavior [GO:0032538], regulation of circadian sleep/wake cycle [GO:0042749], regulation of egg-laying behavior [GO:0046662], positive regulation of behavior [GO:0048520], GO:0048521, regulation of feeding behavior [GO:0060259], regulation of locomotion involved in locomotory behavior [GO:0090325], regulation of olfactory learning [GO:0090328], regulation of male mating behavior [GO:1902435], regulation of foraging behavior [GO:1903368], regulation of locomotor rhythm [GO:1904059], regulation of mechanosensory behavior [GO:1905790], regulation of grooming behavior [GO:2000821], GO:2000822